hydroxyjasmonate sulfotransferase activity [GO:0080131] (molecular function) Also known as: OHJA sulfotransferase activity, hydroxyjasmonic acid sulfotransferase activity, 11-OHJA sulfotransferase activity, 11-hydroxyjasmonate sulfotransferase activity, 11-hydroxyjasmonic acid sulfotransferase activity, 12-OHJA sulfotransferase activity, 12-hydroxyjasmonate sulfotransferase activity, 12-hydroxyjasmonic acid sulfotransferase activity Relationships: is a type of sulfotransferase activity [GO:0008146] Definition: Catalysis of the reaction: a hydroxyjasmonate + 3'-phosphoadenosine-5'-phosphosulfate = a hydroxyjasmonate sulfate + adenosine-3',5'-diphosphate. References: PMID:12637544 Sources: EC:2.8.2.39